{
  "gene": "UniProtKB:Q96RF0",
  "term_id": "GO:0035091",
  "gene_name": "Sorting nexin-18",
  "gene_symbol": "SNX18",
  "term_label": "phosphatidylinositol binding"
}